{
  "term_id": "GO:0004222",
  "gene_name": "Neurolysin, mitochondrial",
  "term_label": "metalloendopeptidase activity",
  "gene_symbol": "NLN",
  "gene": "UniProtKB:Q9BYT8"
}